{
  "gene_symbol": "SLC5A7",
  "term_id": "GO:0045202",
  "gene": "UniProtKB:Q9GZV3",
  "gene_name": "High affinity choline transporter 1",
  "term_label": "synapse"
}